{
  "gene": "UniProtKB:O60641",
  "term_id": "GO:0005905",
  "term_label": "clathrin-coated pit",
  "gene_name": "Clathrin coat assembly protein AP180",
  "gene_symbol": "SNAP91"
}